vitamin D3 25-hydroxylase activity [GO:0030343] (molecular function) Also known as: cholecalciferol 25-hydroxylase activity Relationships: is a type of steroid hydroxylase activity [GO:0008395]; is part of GO:0036378 Definition: Catalysis of the reaction: calciol (vitamin D3) + reduced [NADPH--hemoprotein reductase] + O2 = calcidiol + oxidized [NADPH--hemoprotein reductase] + H2O + H+. Sources: RHEA:32903